{
  "term_label": "somatostatin receptor activity",
  "gene_symbol": "SSTR4",
  "gene": "UniProtKB:P31391",
  "gene_name": "Somatostatin receptor type 4",
  "term_id": "GO:0004994"
}